{
  "term_label": "interleukin-2 receptor binding",
  "term_id": "GO:0005134",
  "gene_name": "Interleukin-2",
  "gene": "UniProtKB:P60568",
  "gene_symbol": "IL2"
}